{
  "term_id": "GO:0031410",
  "term_label": "cytoplasmic vesicle",
  "gene": "UniProtKB:Q6UWJ8",
  "gene_symbol": "CD164L2",
  "gene_name": "CD164 sialomucin-like 2 protein"
}